regulation of melanosome transport [GO:1902908] (biological process) Subtypes: negative regulation of melanosome transport [GO:1902909], positive regulation of melanosome transport [GO:1902910] Relationships: is a type of regulation of cellular process [GO:0050794]; is a type of GO:0051049; regulates melanosome transport [GO:0032402] Definition: Any process that modulates the frequency, rate or extent of melanosome transport. References: PMID:23334344 Sources: GOC:TermGenie, GOC:als, GO_REF:0000058